{
  "gene_name": "Partitioning defective 6 homolog alpha",
  "gene_symbol": "PARD6A",
  "term_label": "Unknown molecular function",
  "term_id": "UNKNOWN:0001",
  "gene": "UniProtKB:Q9NPB6"
}